{
  "gene_symbol": "MCOLN2",
  "gene": "UniProtKB:Q8IZK6",
  "term_label": "Unknown biological process",
  "term_id": "UNKNOWN:0002",
  "gene_name": "Mucolipin-2"
}